{
  "gene_symbol": "CYFIP1",
  "term_id": "GO:0043005",
  "gene_name": "Cytoplasmic FMR1-interacting protein 1",
  "term_label": "neuron projection",
  "gene": "UniProtKB:Q7L576"
}